{
  "term_id": "GO:0019005",
  "gene_name": "F-box only protein 6",
  "gene": "UniProtKB:Q9NRD1",
  "gene_symbol": "FBXO6",
  "term_label": "SCF ubiquitin ligase complex"
}